{
  "term_label": "Unknown molecular function",
  "gene": "UniProtKB:Q8N8F7",
  "gene_name": "Leucine-rich single-pass membrane protein 1",
  "term_id": "UNKNOWN:0001",
  "gene_symbol": "LSMEM1"
}